{
  "term_id": "GO:0050821",
  "gene_name": "Tripartite motif-containing protein 44",
  "gene": "UniProtKB:Q96DX7",
  "gene_symbol": "TRIM44",
  "term_label": "protein stabilization"
}